{
  "term_label": "regulation of transcription by RNA polymerase II",
  "gene_symbol": "ATXN7L3",
  "gene_name": "Ataxin-7-like protein 3",
  "gene": "UniProtKB:Q14CW9",
  "term_id": "GO:0006357"
}